{
  "term_label": "Unknown biological process",
  "gene": "UniProtKB:Q9UK80",
  "gene_name": "Ubiquitin carboxyl-terminal hydrolase 21",
  "term_id": "UNKNOWN:0002",
  "gene_symbol": "USP21"
}